{
  "gene_symbol": "SNCA",
  "term_id": "GO:0001963",
  "term_label": "synaptic transmission, dopaminergic",
  "gene_name": "Alpha-synuclein",
  "gene": "UniProtKB:P37840"
}